{
  "gene": "UniProtKB:X6R8R1",
  "term_label": "SNARE binding",
  "gene_symbol": "SYT15B",
  "gene_name": "Synaptotagmin-15B",
  "term_id": "GO:0000149"
}